{
  "gene": "UniProtKB:O60763",
  "gene_symbol": "USO1",
  "gene_name": "General vesicular transport factor p115",
  "term_label": "intracellular protein transport",
  "term_id": "GO:0006886"
}